{
  "gene_symbol": "LIN7B",
  "gene": "UniProtKB:Q9HAP6",
  "term_id": "GO:0016323",
  "term_label": "basolateral plasma membrane",
  "gene_name": "Protein lin-7 homolog B"
}